{
  "term_id": "GO:0005886",
  "term_label": "plasma membrane",
  "gene": "UniProtKB:P0DQD5",
  "gene_symbol": "NPY4R2",
  "gene_name": "Neuropeptide Y receptor type 4-2"
}